{
  "term_id": "GO:0032720",
  "gene": "UniProtKB:P17213",
  "term_label": "negative regulation of tumor necrosis factor production",
  "gene_symbol": "BPI",
  "gene_name": "Bactericidal permeability-increasing protein"
}